{
  "gene_name": "Homeobox protein DBX1",
  "term_label": "Unknown cellular component",
  "term_id": "UNKNOWN:0003",
  "gene": "UniProtKB:A6NMT0",
  "gene_symbol": "DBX1"
}